{
  "gene_name": "Kinesin-like protein KIF1B",
  "gene_symbol": "KIF1B",
  "term_label": "axon",
  "term_id": "GO:0030424",
  "gene": "UniProtKB:O60333"
}